regulation of skeletal muscle contraction by action potential [GO:0100001] (biological process) Regulation: regulated by GO:0014861 Sources: GOC:cjm, GOC:obol Definition: Any action potential process that regulates skeletal muscle contraction. Relationships: is a type of action potential [GO:0001508]; is a type of regulation of skeletal muscle contraction [GO:0014819]